{
  "gene_name": "N-acetylneuraminate lyase",
  "term_id": "GO:0008747",
  "gene": "UniProtKB:Q9BXD5",
  "term_label": "N-acetylneuraminate lyase activity",
  "gene_symbol": "NPL"
}